{
  "gene_name": "Serine_threonine-protein kinase Nek1",
  "term_id": "UNKNOWN:0002",
  "gene_symbol": "NEK1",
  "gene": "UniProtKB:Q96PY6",
  "term_label": "Unknown biological process"
}